prostaglandin F synthase activity [GO:0047017] (molecular function) Relationships: is a type of oxidoreductase activity, acting on the CH-OH group of donors, NAD or NADP as acceptor [GO:0016616] Also known as: (5Z,13E)-(15S)-9alpha,11alpha,15-trihydroxyprosta-5,13-dienoate:NADP+ 11-oxidoreductase activity, NADPH-dependent prostaglandin D2 11-keto reductase activity, PGD(2) 11-ketoreductase activity, PGD2 11-ketoreductase activity, PGF synthetase activity, PGF2alpha synthetase activity, prostaglandin 11-keto reductase activity, prostaglandin 11-ketoreductase activity, prostaglandin D2-ketoreductase activity, prostaglandin F synthetase activity, prostaglandin-D(2) 11-ketoreductase activity, prostaglandin-D(2) 11-reductase activity, prostaglandin-D(2) ketoreductase activity, prostaglandin-D2 11-ketoreductase activity, prostaglandin-D2 11-reductase activity, prostaglandin-D2 ketoreductase activity, prostaglandin-F synthase activity, prostaglandin-F synthetase activity, reductase, 15-hydroxy-11-oxoprostaglandin, synthetase, prostaglandin F2alpha Definition: Catalysis of the reaction: NADP+ + prostaglandin F2alpha = H+ + NADPH + prostaglandin D2. Sources: RHEA:10140